{
  "gene_name": "Protein PBDC1",
  "term_label": "Unknown cellular component",
  "gene": "UniProtKB:Q9BVG4",
  "term_id": "UNKNOWN:0003",
  "gene_symbol": "PBDC1"
}